{
  "term_id": "GO:0006614",
  "gene_symbol": "SEC63",
  "term_label": "SRP-dependent cotranslational protein targeting to membrane",
  "gene": "UniProtKB:Q9UGP8",
  "gene_name": "Translocation protein SEC63 homolog"
}